{
  "term_id": "GO:0009952",
  "gene_name": "Class E basic helix-loop-helix protein 40",
  "gene_symbol": "BHLHE40",
  "term_label": "anterior/posterior pattern specification",
  "gene": "UniProtKB:O14503"
}